hyaluronan synthase activity [GO:0050501] (molecular function) Definition: Catalysis of the reaction: UDP-D-glucuronate + UDP-N-acetyl-D-glucosamine = [beta-N-acetyl-D-glucosaminyl-(1->4)-beta-D-glucuronosyl-(1->3)](n) + 2n UDP. Relationships: is a type of UDP-glycosyltransferase activity [GO:0008194]; is a type of hexosyltransferase activity [GO:0016758] Also known as: HAS activity, alternating UDP-alpha-N-acetyl-D-glucosamine:beta-D-glucuronosyl-(1,3)-[nascent hyaluronan] 4-N-acetyl-beta-D-glucosaminyltransferase and UDP-alpha-D-glucuronate:N-acetyl-beta-D-glucosaminyl-(1,4)-[nascent hyaluronan] 3-beta-D-glucuronosyltransferase activity, alternating UDP-alpha-N-acetyl-D-glucosamine:beta-D-glucuronosyl-(1->3)-[nascent hyaluronan] 4-N-acetyl-beta-D-glucosaminyltransferase and UDP-alpha-D-glucuronate:N-acetyl-beta-D-glucosaminyl-(1->4)-[nascent hyaluronan] 3-beta-D-glucuronosyltransferase activity, seHAS, spHAS Sources: EC:2.4.1.212, MetaCyc:2.4.1.212-RXN